{
  "term_id": "UNKNOWN:0001",
  "gene_symbol": "RNF32",
  "gene_name": "RING finger protein 32",
  "term_label": "Unknown molecular function",
  "gene": "UniProtKB:Q9H0A6"
}